{
  "term_id": "GO:0005829",
  "gene_symbol": "AHCY",
  "gene_name": "Adenosylhomocysteinase",
  "gene": "UniProtKB:P23526",
  "term_label": "cytosol"
}